{
  "gene_name": "Molybdenum cofactor biosynthesis protein 1",
  "gene_symbol": "MOCS1",
  "term_label": "GTP 3',8'-cyclase activity",
  "term_id": "GO:0061798",
  "gene": "UniProtKB:Q9NZB8"
}